{
  "term_id": "GO:0005044",
  "term_label": "scavenger receptor activity",
  "gene": "UniProtKB:Q4G0T1",
  "gene_symbol": "SCART1",
  "gene_name": "Scavenger receptor cysteine-rich domain-containing protein SCART1"
}